{
  "gene_name": "Carnitine O-palmitoyltransferase 2, mitochondrial",
  "gene": "UniProtKB:P23786",
  "term_id": "GO:0006635",
  "term_label": "fatty acid beta-oxidation",
  "gene_symbol": "CPT2"
}